{
  "term_id": "GO:0006357",
  "gene": "UniProtKB:Q96K83",
  "term_label": "regulation of transcription by RNA polymerase II",
  "gene_name": "Zinc finger protein 521",
  "gene_symbol": "ZNF521"
}